{
  "gene_name": "SEC14 domain and spectrin repeat-containing protein 1",
  "term_label": "phosphatidylinositol-5-phosphate binding",
  "gene_symbol": "SESTD1",
  "gene": "UniProtKB:Q86VW0",
  "term_id": "GO:0010314"
}